{
  "term_label": "Unknown cellular component",
  "gene": "UniProtKB:Q8N535",
  "gene_name": "Putative uncharacterized protein encoded by LINC00471",
  "gene_symbol": "LINC00471",
  "term_id": "UNKNOWN:0003"
}